{
  "gene_name": "Disintegrin and metalloproteinase domain-containing protein 11",
  "gene": "UniProtKB:O75078",
  "term_id": "UNKNOWN:0003",
  "term_label": "Unknown cellular component",
  "gene_symbol": "ADAM11"
}